{
  "gene_name": "Putative zinc finger protein 487",
  "term_id": "GO:0005634",
  "gene": "UniProtKB:B1APH4",
  "gene_symbol": "ZNF487",
  "term_label": "nucleus"
}